{
  "gene_symbol": "ARF6",
  "term_id": "GO:0006886",
  "gene_name": "ADP-ribosylation factor 6",
  "term_label": "intracellular protein transport",
  "gene": "UniProtKB:P62330"
}